{
  "term_id": "GO:0160203",
  "gene_name": "Apoptosis-inducing factor 1, mitochondrial",
  "term_label": "mitochondrial disulfide relay system",
  "gene": "UniProtKB:O95831",
  "gene_symbol": "AIFM1"
}